{
  "term_label": "filamentous actin",
  "gene_symbol": "LDB3",
  "term_id": "GO:0031941",
  "gene": "UniProtKB:O75112",
  "gene_name": "LIM domain-binding protein 3"
}